{
  "term_label": "extracellular space",
  "gene_symbol": "ADAM9",
  "term_id": "GO:0005615",
  "gene_name": "Disintegrin and metalloproteinase domain-containing protein 9",
  "gene": "UniProtKB:Q13443"
}